{
  "gene_name": "Putative metallothionein MT1DP",
  "gene": "UniProtKB:A1L3X4",
  "gene_symbol": "MT1DP",
  "term_id": "GO:0071276",
  "term_label": "cellular response to cadmium ion"
}